brush border membrane [GO:0031526] (cellular component) Definition: The portion of the plasma membrane surrounding the brush border. Sources: GOC:mah Relationships: is a type of cell projection membrane [GO:0031253]; is part of GO:0005903; is part of GO:0016324